{
  "gene": "UniProtKB:Q9UP38",
  "gene_name": "Frizzled-1",
  "term_label": "non-canonical Wnt signaling pathway",
  "term_id": "GO:0035567",
  "gene_symbol": "FZD1"
}